response to leptomycin B [GO:1901344] (biological process) Subtypes: cellular response to leptomycin B [GO:0072750] Relationships: is a type of response to fatty acid [GO:0070542] Sources: GOC:TermGenie Definition: Any process that results in a change in state or activity of a cell or an organism (in terms of movement, secretion, enzyme production, gene expression, etc.) as a result of a leptomycin B stimulus.